{
  "gene_name": "Glutamate-rich protein 6B",
  "term_id": "UNKNOWN:0003",
  "gene": "UniProtKB:Q5W0A0",
  "term_label": "Unknown cellular component",
  "gene_symbol": "ERICH6B"
}